{
  "gene": "UniProtKB:Q9Y2K1",
  "term_id": "GO:0002682",
  "gene_symbol": "ZBTB1",
  "gene_name": "Zinc finger and BTB domain-containing protein 1",
  "term_label": "regulation of immune system process"
}